{
  "gene_name": "Kinesin-like protein KIF3A",
  "gene_symbol": "KIF3A",
  "term_id": "GO:0003777",
  "gene": "UniProtKB:Q9Y496",
  "term_label": "microtubule motor activity"
}